{
  "gene_name": "Brefeldin A-inhibited guanine nucleotide-exchange protein 1",
  "term_id": "GO:0005085",
  "term_label": "guanyl-nucleotide exchange factor activity",
  "gene_symbol": "ARFGEF1",
  "gene": "UniProtKB:Q9Y6D6"
}